positive regulation of inosine transport [GO:0035342] (biological process) Sources: GOC:bf Also known as: positive regulation of hypoxanthine riboside transport Definition: Any process that activates or increases the frequency, rate or extent of the directed movement of inosine into, out of or within a cell, or between cells, by means of some agent such as a transporter or pore. Relationships: is a type of positive regulation of purine nucleoside transport [GO:0032248]; is a type of regulation of inosine transport [GO:0035341]; positively regulates inosine transport [GO:0035340]